{
  "gene": "UniProtKB:Q9BZB8",
  "term_id": "GO:0000900",
  "gene_name": "Cytoplasmic polyadenylation element-binding protein 1",
  "gene_symbol": "CPEB1",
  "term_label": "mRNA regulatory element binding translation repressor activity"
}